{
  "term_id": "GO:0005615",
  "gene_symbol": "LCN2",
  "gene": "UniProtKB:P80188",
  "gene_name": "Neutrophil gelatinase-associated lipocalin",
  "term_label": "extracellular space"
}